{
  "gene_name": "Otolin-1",
  "gene_symbol": "OTOL1",
  "term_id": "UNKNOWN:0003",
  "gene": "UniProtKB:A6NHN0",
  "term_label": "Unknown cellular component"
}